{
  "gene": "UniProtKB:Q13490",
  "term_label": "ubiquitin protein ligase activity",
  "term_id": "GO:0061630",
  "gene_name": "Baculoviral IAP repeat-containing protein 2",
  "gene_symbol": "BIRC2"
}